{
  "term_id": "GO:0000785",
  "term_label": "chromatin",
  "gene": "UniProtKB:Q9ULJ6",
  "gene_symbol": "ZMIZ1",
  "gene_name": "Zinc finger MIZ domain-containing protein 1"
}